{
  "gene_name": "Nuclear factor of activated T-cells, cytoplasmic 2",
  "gene_symbol": "NFATC2",
  "gene": "UniProtKB:Q13469",
  "term_label": "DNA-binding transcription factor activity, RNA polymerase II-specific",
  "term_id": "GO:0000981"
}